{
  "gene": "UniProtKB:Q96RF0",
  "gene_name": "Sorting nexin-18",
  "term_label": "endocytosis",
  "gene_symbol": "SNX18",
  "term_id": "GO:0006897"
}